{
  "gene_symbol": "CA13",
  "gene_name": "Carbonic anhydrase 13",
  "gene": "UniProtKB:Q8N1Q1",
  "term_id": "GO:0005737",
  "term_label": "cytoplasm"
}